{
  "term_label": "DNA-binding transcription factor activity, RNA polymerase II-specific",
  "gene_name": "Zinc finger and SCAN domain-containing protein 20",
  "gene": "UniProtKB:P17040",
  "gene_symbol": "ZSCAN20",
  "term_id": "GO:0000981"
}